{
  "gene": "UniProtKB:A8MUN3",
  "gene_symbol": "A8MUN3",
  "term_label": "Unknown molecular function",
  "term_id": "UNKNOWN:0001",
  "gene_name": "Putative uncharacterized protein ENSP00000381830"
}